negative regulation of hematopoietic stem cell migration [GO:2000472] (biological process) Definition: Any process that stops, prevents or reduces the frequency, rate or extent of hematopoietic stem cell migration. Also known as: negative regulation of hemopoietic stem cell migration Sources: GOC:obol Relationships: is a type of negative regulation of cell migration [GO:0030336]; is a type of regulation of hematopoietic stem cell migration [GO:2000471]; negatively regulates GO:0035701